histone H3K18cr reader activity [GO:0140017] (molecular function) Definition: A histone reader that recognizes a histone H3 crotonylated at lysine 18. References: PMID:27105114 Also known as: H3K18cr modified histone binding Note: Comment: Note that the residue position corresponds to the canonical human H3 histone (UniProtKB:P84243); this residue is conserved across all eukaryotes. Residue 1 is the first residue following removal of the initiating Methionine (Met). Note that each histone is encoded by multiple genes, and sequences may vary across different genes within an organism. Relationships: is a type of histone H3 reader activity [GO:0140006]